{
  "term_label": "ribosome binding",
  "gene_name": "Translation initiation factor IF-3, mitochondrial",
  "gene_symbol": "MTIF3",
  "term_id": "GO:0043022",
  "gene": "UniProtKB:Q9H2K0"
}